{
  "gene": "UniProtKB:Q9BT22",
  "gene_name": "Chitobiosyldiphosphodolichol beta-mannosyltransferase",
  "gene_symbol": "ALG1",
  "term_label": "endoplasmic reticulum",
  "term_id": "GO:0005783"
}